{
  "gene_symbol": "ERV3-1",
  "term_id": "UNKNOWN:0001",
  "term_label": "Unknown molecular function",
  "gene": "UniProtKB:Q14264",
  "gene_name": "Endogenous retrovirus group 3 member 1 Env polyprotein"
}